metanephric juxtaglomerulus cell fate commitment [GO:0072253] (biological process) Definition: The process in which the developmental fate of a cell becomes restricted such that it will develop into a metanephric juxtaglomerulus cell. Sources: GOC:mtg_kidney_jan10 Relationships: is a type of GO:0072150; is part of GO:0072251